chemosensory jump behavior [GO:0007636] (biological process) Definition: The sudden, usually upward, movement off the ground or other surface through sudden muscular effort in the legs, following exposure to a chemical substance. Relationships: is a type of jump response [GO:0007630]; is a type of chemosensory behavior [GO:0007635] Also known as: chemosensory jump behaviour, jump response to chemical stimulus Sources: GOC:jid